{
  "gene": "UniProtKB:O60225",
  "gene_symbol": "SSX5",
  "term_label": "nucleus",
  "gene_name": "Protein SSX5",
  "term_id": "GO:0005634"
}